{
  "gene_symbol": "ADPGK",
  "term_id": "GO:0006006",
  "term_label": "glucose metabolic process",
  "gene_name": "ADP-dependent glucokinase",
  "gene": "UniProtKB:Q9BRR6"
}